{
  "term_id": "GO:0005743",
  "gene_name": "5-demethoxyubiquinone hydroxylase, mitochondrial",
  "gene_symbol": "COQ7",
  "term_label": "mitochondrial inner membrane",
  "gene": "UniProtKB:Q99807"
}